type 1 member 3 taste receptor binding [GO:0031886] (molecular function) Definition: Binding to a type 1 member 3 taste receptor. Also known as: sweet taste receptor binding, type 1 member 3 taste receptor ligand Sources: GOC:mah, GOC:nln Relationships: is a type of GO:0031883